{
  "gene": "UniProtKB:P42694",
  "term_id": "GO:0003723",
  "term_label": "RNA binding",
  "gene_name": "Probable helicase with zinc finger domain",
  "gene_symbol": "HELZ"
}